{
  "gene_name": "Nitric oxide synthase-interacting protein",
  "term_label": "nucleus",
  "gene_symbol": "NOSIP",
  "gene": "UniProtKB:Q9Y314",
  "term_id": "GO:0005634"
}